{
  "gene_name": "Etoposide-induced protein 2.4 homolog",
  "term_label": "endoplasmic reticulum",
  "gene": "UniProtKB:O14681",
  "gene_symbol": "EI24",
  "term_id": "GO:0005783"
}